{
  "gene_symbol": "IVNS1ABP",
  "gene": "UniProtKB:Q9Y6Y0",
  "term_label": "ubiquitin-like ligase-substrate adaptor activity",
  "gene_name": "Influenza virus NS1A-binding protein",
  "term_id": "GO:1990756"
}